{
  "gene_name": "T cell receptor beta variable 4-3",
  "term_label": "cell surface receptor signaling pathway",
  "term_id": "GO:0007166",
  "gene": "UniProtKB:A0A589",
  "gene_symbol": "TRBV4-3"
}